{
  "term_label": "chromatin",
  "gene_name": "Protein HIRA",
  "gene_symbol": "HIRA",
  "gene": "UniProtKB:P54198",
  "term_id": "GO:0000785"
}